{
  "term_id": "GO:0010468",
  "term_label": "regulation of gene expression",
  "gene": "UniProtKB:A6NK02",
  "gene_name": "Tripartite motif-containing protein 75",
  "gene_symbol": "TRIM75"
}